cellular response to vitamin B2 [GO:0071302] (biological process) Sources: GOC:mah Also known as: cellular response to riboflavin Definition: Any process that results in a change in state or activity of a cell (in terms of movement, secretion, enzyme production, gene expression, etc.) as a result of a vitamin B2 stimulus. Relationships: is a type of response to vitamin B2 [GO:0033274]; is a type of cellular response to vitamin [GO:0071295]; is a type of cellular response to nitrogen compound [GO:1901699]; is a type of cellular response to oxygen-containing compound [GO:1901701]